{
  "term_id": "GO:0008021",
  "gene": "UniProtKB:P51790",
  "term_label": "synaptic vesicle",
  "gene_symbol": "CLCN3",
  "gene_name": "H(+)_Cl(-) exchange transporter 3"
}